{
  "term_label": "heme binding",
  "term_id": "GO:0020037",
  "gene_symbol": "CYB5R4",
  "gene": "UniProtKB:Q7L1T6",
  "gene_name": "Cytochrome b5 reductase 4"
}